{
  "gene": "UniProtKB:P02708",
  "term_label": "acetylcholine-gated channel complex",
  "term_id": "GO:0005892",
  "gene_name": "Acetylcholine receptor subunit alpha",
  "gene_symbol": "CHRNA1"
}